{
  "term_id": "GO:0007165",
  "gene_symbol": "OR7G3",
  "gene_name": "Olfactory receptor 7G3",
  "gene": "UniProtKB:Q8NG95",
  "term_label": "signal transduction"
}